{
  "gene_symbol": "SNRPGP15",
  "gene_name": "Putative small nuclear ribonucleoprotein G-like protein 15",
  "term_id": "GO:0005689",
  "gene": "UniProtKB:A8MWD9",
  "term_label": "U12-type spliceosomal complex"
}